{
  "term_id": "UNKNOWN:0001",
  "gene": "UniProtKB:Q96IK0",
  "term_label": "Unknown molecular function",
  "gene_symbol": "TMEM101",
  "gene_name": "Transmembrane protein 101"
}